{
  "term_label": "regulation of cell cycle process",
  "term_id": "GO:0010564",
  "gene": "UniProtKB:Q01101",
  "gene_symbol": "INSM1",
  "gene_name": "Insulinoma-associated protein 1"
}